negative regulation of aspartate secretion [GO:1904449] (biological process) Relationships: is a type of negative regulation of organic acid transport [GO:0032891]; is a type of negative regulation of amino acid transport [GO:0051956]; is a type of negative regulation of secretion by cell [GO:1903531]; is a type of regulation of aspartate secretion [GO:1904448]; negatively regulates aspartate secretion [GO:0061528] Also known as: down regulation of aspartate secretion, down-regulation of aspartate secretion, downregulation of aspartate secretion, inhibition of aspartate secretion Definition: Any process that stops, prevents or reduces the frequency, rate or extent of aspartate secretion. References: PMID:2342602 Sources: GOC:TermGenie, GO_REF:0000058